{
  "gene": "UniProtKB:Q5JTY5",
  "term_id": "GO:0008270",
  "gene_symbol": "ZNG1C",
  "term_label": "zinc ion binding",
  "gene_name": "Zinc-regulated GTPase metalloprotein activator 1C"
}